positive regulation of establishment or maintenance of bipolar cell polarity regulating cell shape [GO:2000247] (biological process) Relationships: is a type of regulation of establishment or maintenance of bipolar cell polarity regulating cell shape [GO:2000100]; is a type of positive regulation of establishment or maintenance of cell polarity regulating cell shape [GO:2000771]; positively regulates establishment or maintenance of bipolar cell polarity regulating cell shape [GO:0061246] Subtypes: positive regulation of establishment of bipolar cell polarity regulating cell shape [GO:0061161], positive regulation of maintenance of bipolar cell polarity regulating cell shape [GO:0061361] Sources: GOC:obol Definition: Any process that activates or increases the frequency, rate or extent of establishment or maintenance of bipolar cell polarity regulating cell shape.